{
  "gene_name": "Neuroblastoma breakpoint family member 14",
  "term_label": "Unknown molecular function",
  "gene_symbol": "NBPF14",
  "term_id": "UNKNOWN:0001",
  "gene": "UniProtKB:Q5TI25"
}